regulation of inositol trisphosphate biosynthetic process [GO:0032960] (biological process) Sources: GOC:mah Subtypes: negative regulation of inositol trisphosphate biosynthetic process [GO:0032961], GO:0032962 Relationships: is a type of GO:0010919; regulates inositol trisphosphate biosynthetic process [GO:0032959] Definition: Any process that modulates the frequency, rate or extent of the chemical reactions and pathways resulting in the formation of inositol trisphosphate. Also known as: regulation of IP3 biosynthesis, regulation of IP3 biosynthetic process, regulation of inositol trisphosphate anabolism, regulation of inositol trisphosphate biosynthesis, regulation of inositol trisphosphate formation, regulation of inositol trisphosphate synthesis, regulation of myo-inositol trisphosphate biosynthesis, regulation of myo-inositol trisphosphate biosynthetic process